{
  "term_label": "Unknown biological process",
  "gene_symbol": "GAS8-AS1",
  "term_id": "UNKNOWN:0002",
  "gene": "UniProtKB:O95177",
  "gene_name": "Uncharacterized protein GAS8-AS1"
}